{
  "gene_name": "Lamin-B2",
  "gene_symbol": "LMNB2",
  "term_id": "GO:0090435",
  "term_label": "protein localization to nuclear envelope",
  "gene": "UniProtKB:Q03252"
}